{
  "term_id": "GO:0005783",
  "gene_symbol": "PDIA5",
  "term_label": "endoplasmic reticulum",
  "gene": "UniProtKB:Q14554",
  "gene_name": "Protein disulfide-isomerase A5"
}